regulation of protein-pyridoxal-5-phosphate linkage [GO:1904285] (biological process) Relationships: is a type of GO:0031399; regulates protein-pyridoxal-5-phosphate linkage [GO:0018352] References: PMID:25957689 Sources: GOC:TermGenie, GO_REF:0000058 Definition: Any process that modulates the frequency, rate or extent of protein-pyridoxal-5-phosphate linkage. Subtypes: negative regulation of protein-pyridoxal-5-phosphate linkage [GO:1904286], GO:1904287